{
  "gene": "UniProtKB:P42338",
  "term_id": "GO:0005886",
  "term_label": "plasma membrane",
  "gene_symbol": "PIK3CB",
  "gene_name": "Phosphatidylinositol 4,5-bisphosphate 3-kinase catalytic subunit beta isoform"
}